{
  "term_label": "Cul2-RING ubiquitin ligase complex",
  "gene_name": "PRAME family member 5",
  "gene": "UniProtKB:Q5TYX0",
  "gene_symbol": "PRAMEF5",
  "term_id": "GO:0031462"
}